spectrin binding [GO:0030507] (MF) Sources: GOC:mah, ISBN:0198506732 Definition: Binding to spectrin, a protein that is the major constituent of the erythrocyte cytoskeletal network. It associates with band 4.1 (see band protein) and actin to form the cytoskeletal superstructure of the erythrocyte plasma membrane. It is composed of nonhomologous chains, alpha and beta, which aggregate side-to-side in an antiparallel fashion to form dimers, tetramers, and higher polymers. Relationships: is a type of GO:0008092; is a type of protein-containing complex binding [GO:0044877]